{
  "gene": "UniProtKB:Q7Z2Y8",
  "term_label": "Unknown cellular component",
  "term_id": "UNKNOWN:0003",
  "gene_symbol": "GVINP1",
  "gene_name": "Interferon-induced very large GTPase 1"
}